{
  "gene_symbol": "SNX2",
  "gene_name": "Sorting nexin-2",
  "gene": "UniProtKB:O60749",
  "term_label": "endosome membrane",
  "term_id": "GO:0010008"
}